{
  "gene_symbol": "BRICD5",
  "gene_name": "BRICHOS domain-containing protein 5",
  "term_label": "regulation of cell population proliferation",
  "term_id": "GO:0042127",
  "gene": "UniProtKB:Q6PL45"
}